{
  "gene_symbol": "PACSIN3",
  "term_label": "phospholipid binding",
  "term_id": "GO:0005543",
  "gene_name": "Protein kinase C and casein kinase substrate in neurons protein 3",
  "gene": "UniProtKB:Q9UKS6"
}